{
  "gene_symbol": "FBXL19",
  "term_label": "histone demethylase activity",
  "gene_name": "F-box_LRR-repeat protein 19",
  "gene": "UniProtKB:Q6PCT2",
  "term_id": "GO:0032452"
}